protein K27-linked ubiquitination [GO:0044314] (biological process) References: PMID:19345326 Also known as: protein K27-linked polyubiquitination Definition: A protein ubiquitination process in which a polymer of ubiquitin, formed by linkages between lysine residues at position 27 of the ubiquitin monomers, is added to a protein. Relationships: is a type of GO:0000209